positive regulation of sterol biosynthetic process [GO:0106120] (biological process) Relationships: is a type of positive regulation of steroid biosynthetic process [GO:0010893]; is a type of GO:0106118; positively regulates sterol biosynthetic process [GO:0016126] Subtypes: positive regulation of cholesterol biosynthetic process [GO:0045542], GO:0070452 Definition: Any process that activates or increases the frequency, rate or extent of a sterol biosynthetic process. References: PMID:16459310 Sources: GOC:BHF, GOC:BHF_miRNA, GOC:rph